inositol-1,3,4,5-tetrakisphosphate 5-phosphatase activity [GO:0052659] (molecular function) Definition: Catalysis of the reaction: 1D-myo-inositol 1,3,4,5-tetrakisphosphate + H2O = 1D-myo-inositol 1,3,4-trisphosphate + phosphate. Sources: RHEA:11392 Relationships: is a type of inositol-polyphosphate 5-phosphatase activity [GO:0004445]; is_a GO:0052743 Also known as: inositol polyphosphate-5-phosphatase activity, D-myo-inositol (1,3,4,5)-polyphosphate 5-phosphatase activity, Ins(1,3,4,5)P(4) 5-phosphatase activity, Ins(1,3,4,5)P4 5-phosphatase activity, type I inositol-polyphosphate phosphatase activity, type II inositol polyphosphate 5-phosphatase activity